{
  "gene_symbol": "ICA1L",
  "term_id": "GO:0051046",
  "gene": "UniProtKB:Q8NDH6",
  "gene_name": "Islet cell autoantigen 1-like protein",
  "term_label": "regulation of secretion"
}